group III metabotropic glutamate receptor activity [GO:0001642] (molecular function) Relationships: is a type of adenylate cyclase inhibiting G protein-coupled glutamate receptor activity [GO:0001640] References: PMID:9016303 Definition: A G protein-coupled receptor that is activated by L-AP-4 and inhibits adenylate cyclase activity.